regulation of mitotic cell cycle [GO:0007346] (biological process) Definition: Any process that modulates the rate or extent of progress through the mitotic cell cycle. Relationships: is a type of regulation of cell cycle [GO:0051726]; RO_0002211 GO:0000278 Subtypes: GO:0007088, regulation of mitotic cell cycle, embryonic [GO:0009794], negative regulation of mitotic cell cycle [GO:0045930], positive regulation of mitotic cell cycle [GO:0045931], regulation of cell cycle switching, mitotic to meiotic cell cycle [GO:0110044], regulation of mitotic cell cycle phase transition [GO:1901990], regulation of mitotic cell cycle DNA replication [GO:1903463], regulation of mitotic spindle checkpoint [GO:1903504], GO:1904289 Also known as: mitotic cell cycle modulation, mitotic cell cycle regulation, modulation of mitotic cell cycle progression, regulation of mitotic cell cycle progression, regulation of progression through mitotic cell cycle, mitotic cell cycle regulator Sources: GOC:dph, GOC:go_curators, GOC:tb